{
  "gene_name": "Integrin alpha-6",
  "term_label": "integrin alpha6-beta1 complex",
  "gene_symbol": "ITGA6",
  "gene": "UniProtKB:P23229",
  "term_id": "GO:0034675"
}